{
  "gene": "UniProtKB:Q9UNX4",
  "gene_symbol": "WDR3",
  "term_id": "GO:0034388",
  "term_label": "Pwp2p-containing subcomplex of 90S preribosome",
  "gene_name": "WD repeat-containing protein 3"
}